cellular response to absence of light [GO:0071485] (biological process) Subtypes: dark adaptation [GO:1990603] Sources: GOC:mah Definition: Any process that results in a change in state or activity of a cell (in terms of movement, secretion, enzyme production, gene expression, etc.) as a result of an absence of light stimuli. Relationships: is a type of response to absence of light [GO:0009646]; is a type of cellular response to light intensity [GO:0071484] Also known as: cellular response to darkness